negative regulation of T-helper cell differentiation [GO:0045623] (biological process) Definition: Any process that stops, prevents, or reduces the frequency, rate or extent of T-helper cell differentiation. Sources: GOC:go_curators Also known as: down regulation of T-helper cell differentiation, down-regulation of T-helper cell differentiation, downregulation of T-helper cell differentiation, inhibition of T-helper cell differentiation, negative regulation of T-helper cell development Note: Note that immunologists typically use the word 'development' to refer to cells of B or T cell lineages undergoing the process that GO describes as 'cell differentiation'. Relationships: is a type of negative regulation of immune effector process [GO:0002698]; is a type of negative regulation of CD4-positive, alpha-beta T cell differentiation [GO:0043371]; is a type of regulation of T-helper cell differentiation [GO:0045622]; is a type of negative regulation of immune response [GO:0050777]; negatively regulates GO:0042093 Subtypes: negative regulation of T-helper 1 cell differentiation [GO:0045626], GO:0045629, negative regulation of T-helper 17 cell differentiation [GO:2000320]